methyltransferase regulator activity [GO:0141107] (molecular function) Subtypes: GO:0141106 Definition: Binds to and modulates the activity of a methyltransferase. References: PMID:15899842, PMID:34669960 Relationships: is a type of enzyme regulator activity [GO:0030234]; regulates methyltransferase activity [GO:0008168]